{
  "gene": "UniProtKB:Q9NZ56",
  "term_id": "GO:0005634",
  "gene_name": "Formin-2",
  "gene_symbol": "FMN2",
  "term_label": "nucleus"
}